{
  "gene_name": "Transcriptional activator protein Pur-alpha",
  "gene": "UniProtKB:Q00577",
  "term_id": "GO:0032422",
  "term_label": "purine-rich negative regulatory element binding",
  "gene_symbol": "PURA"
}